contractile vacuole organization [GO:0033298] (biological process) Definition: A process that is carried out at the cellular level which results in the assembly, arrangement of constituent parts, or disassembly of a contractile vacuole. A specialized vacuole that fills with water from the cytoplasm and then discharges this externally by the opening of contractile vacuole pores. Also known as: contractile vacuole organisation, contractile vacuole organization and biogenesis Relationships: is a type of vacuole organization [GO:0007033]; is a type of vesicle organization [GO:0016050] Sources: GOC:mah